{
  "term_id": "GO:0070888",
  "gene": "UniProtKB:Q8N100",
  "gene_symbol": "ATOH7",
  "gene_name": "Transcription factor ATOH7",
  "term_label": "E-box binding"
}